{
  "term_label": "Unknown cellular component",
  "term_id": "UNKNOWN:0003",
  "gene": "UniProtKB:O15524",
  "gene_symbol": "SOCS1",
  "gene_name": "Suppressor of cytokine signaling 1"
}